{
  "gene": "UniProtKB:Q9NYA1",
  "gene_symbol": "SPHK1",
  "term_label": "cellular response to growth factor stimulus",
  "gene_name": "Sphingosine kinase 1",
  "term_id": "GO:0071363"
}